{
  "term_id": "UNKNOWN:0003",
  "gene_symbol": "CCDC120",
  "gene_name": "Coiled-coil domain-containing protein 120",
  "gene": "UniProtKB:Q96HB5",
  "term_label": "Unknown cellular component"
}